flavone biosynthetic process [GO:0051553] (biological process) Relationships: is a type of flavonoid biosynthetic process [GO:0009813]; is a type of pigment biosynthetic process [GO:0046148]; is a type of flavone metabolic process [GO:0051552] Also known as: 2-phenyl-4H-1-benzopyran-4-one biosynthesis, 2-phenyl-4H-1-benzopyran-4-one biosynthetic process, 2-phenylchromone biosynthesis, 2-phenylchromone biosynthetic process Definition: The chemical reactions and pathways resulting in the formation of flavones, a class of pigmented plant compounds based on 2-phenyl-4H-1-benzopyran-4-one (2-phenylchromone). References: PMID:18567791 Sources: GOC:ai Subtypes: quercetin O-glucoside biosynthetic process [GO:0033303], kaempferol O-glucoside biosynthetic process [GO:0033330], luteolin biosynthetic process [GO:0033511], flavonol biosynthetic process [GO:0051555], quercetin biosynthetic process [GO:1901734]